{
  "term_id": "GO:0035845",
  "gene_name": "Photoreceptor cilium actin regulator",
  "gene_symbol": "PCARE",
  "gene": "UniProtKB:A6NGG8",
  "term_label": "photoreceptor cell outer segment organization"
}